{
  "gene_symbol": "BRCA1",
  "gene_name": "Breast cancer type 1 susceptibility protein",
  "term_id": "GO:0004842",
  "term_label": "ubiquitin-protein transferase activity",
  "gene": "UniProtKB:P38398"
}